{
  "term_id": "GO:0005886",
  "gene": "UniProtKB:Q8IZF6",
  "gene_symbol": "ADGRG4",
  "gene_name": "Adhesion G-protein coupled receptor G4",
  "term_label": "plasma membrane"
}